{
  "gene": "UniProtKB:Q92608",
  "term_id": "GO:0005886",
  "gene_name": "Dedicator of cytokinesis protein 2",
  "term_label": "plasma membrane",
  "gene_symbol": "DOCK2"
}